{
  "gene_symbol": "ZNF782",
  "term_id": "GO:0000976",
  "gene": "UniProtKB:Q6ZMW2",
  "term_label": "transcription cis-regulatory region binding",
  "gene_name": "Zinc finger protein 782"
}